indole metabolic process [GO:0042431] (biological process) Also known as: indole metabolism Definition: The chemical reactions and pathways involving indole (2,3-benzopyrrole), the basis of many biologically active substances (e.g. serotonin, tryptophan). Sources: GOC:jl Relationships: is_a GO:0042430 Subtypes: indole biosynthetic process [GO:0042432], indole catabolic process [GO:0042433]